protein-N-terminal amino-acid acetyltransferase activity [GO:0004596] (molecular function) Subtypes: protein-N-terminal-alanine acetyltransferase activity [GO:0008999], protein N-terminal-methionine acetyltransferase activity [GO:0120518], tubulin N-terminal-methionine acetyltransferase activity [GO:0120519], GO:1990189, protein-N-terminal-glutamate acetyltransferase activity [GO:1990190] References: PMID:30054468 Sources: RHEA:21028 Also known as: acetyl-CoA:peptide alpha-N-acetyltransferase activity, acetyl-CoA:peptide nalpha-acetyltransferase activity, nalpha-acetyltransferase activity, peptide alpha-N-acetyltransferase activity, protein N-terminal acetyltransferase activity, beta-endorphin acetyltransferase activity, N(alpha)-acetyltransferase activity, NAT activity, amino-terminal amino acid-acetylating enzyme activity, peptide acetyltransferase activity Relationships: is a type of protein N-acetyltransferase activity [GO:0034212] Definition: Catalysis of the reaction: acetyl-CoA + an N-terminal L-alpha-aminoacyl-[protein] = CoA + H+ + N-terminal Nalpha-acetyl-L-alpha-aminoacyl-[protein].